{
  "gene_name": "F-box_WD repeat-containing protein 4",
  "gene": "UniProtKB:P57775",
  "gene_symbol": "FBXW4",
  "term_id": "UNKNOWN:0001",
  "term_label": "Unknown molecular function"
}